myeloid dendritic cell activation involved in immune response [GO:0002277] (biological process) Definition: The change in morphology and behavior of a myeloid dendritic cell resulting from exposure to a cytokine, chemokine, cellular ligand, or soluble factor, leading to the initiation or perpetuation of an immune response. Sources: GOC:add, ISBN:0781735149 Also known as: myeloid dendritic cell activation during immune response Relationships: is a type of GO:0001773; is a type of myeloid cell activation involved in immune response [GO:0002275] Subtypes: myeloid dendritic cell differentiation involved in immune response [GO:0002284]